{
  "term_label": "polysaccharide biosynthetic process",
  "gene_symbol": "HAS3",
  "term_id": "GO:0000271",
  "gene_name": "Hyaluronan synthase 3",
  "gene": "UniProtKB:O00219"
}